{
  "gene_symbol": "ARSI",
  "gene": "UniProtKB:Q5FYB1",
  "term_id": "UNKNOWN:0003",
  "term_label": "Unknown cellular component",
  "gene_name": "Arylsulfatase I"
}